plasma membrane-derived chromatophore membrane [GO:0042717] (cellular component) Definition: The lipid bilayer associated with a plasma membrane-derived chromatophore; surrounds chromatophores that form complete vesicles. References: PMID:11867431 Sources: GOC:jl, GOC:mah, ISBN:0395825172 Relationships: is a type of GO:0034357; BFO_0000050 GO:0042716 Subtypes: plasma membrane-derived thylakoid membrane [GO:0031676]